{
  "gene_name": "Sorting nexin-4",
  "gene_symbol": "SNX4",
  "term_label": "phosphatidylinositol-3-phosphate binding",
  "term_id": "GO:0032266",
  "gene": "UniProtKB:O95219"
}